{
  "term_id": "GO:0061844",
  "gene_symbol": "PPBP",
  "term_label": "antimicrobial humoral immune response mediated by antimicrobial peptide",
  "gene_name": "Platelet basic protein",
  "gene": "UniProtKB:P02775"
}